{
  "term_id": "GO:0005737",
  "gene_symbol": "AKAP12",
  "gene_name": "A-kinase anchor protein 12",
  "gene": "UniProtKB:Q02952",
  "term_label": "cytoplasm"
}